induced systemic resistance, ethylene mediated signaling pathway [GO:0009866] (biological process) Relationships: is a type of GO:0002218; is a type of immune effector process [GO:0002252]; is a type of ethylene-activated signaling pathway [GO:0009873]; is part of induced systemic resistance [GO:0009682] Sources: GOC:jy Also known as: ethene mediated signaling pathway (induced systemic resistance), ethylene mediated signaling pathway (induced systemic resistance), induced systemic resistance, ethene mediated signaling pathway, induced systemic resistance, ethene mediated signalling pathway, induced systemic resistance, ethylene mediated signalling pathway Definition: The series of molecular signals mediated by ethylene (ethene) involved in induced systemic resistance.